{
  "gene": "UniProtKB:Q96II8",
  "gene_name": "DISP complex protein LRCH3",
  "term_label": "Unknown molecular function",
  "gene_symbol": "LRCH3",
  "term_id": "UNKNOWN:0001"
}